{
  "gene": "UniProtKB:Q9BTC8",
  "gene_name": "Metastasis-associated protein MTA3",
  "term_id": "GO:0000122",
  "term_label": "negative regulation of transcription by RNA polymerase II",
  "gene_symbol": "MTA3"
}